{
  "gene_name": "UDP-glucuronosyltransferase 1A5",
  "gene": "UniProtKB:P35504",
  "term_id": "GO:0019899",
  "term_label": "enzyme binding",
  "gene_symbol": "UGT1A5"
}